anaerobic fatty acid catabolic process [GO:1990486] (biological process) Relationships: is a type of fatty acid catabolic process [GO:0009062] References: PMID:17329794 Sources: GOC:mengo_curators Also known as: anaerobic fatty acid degradation Definition: The chemical reactions and pathways resulting in the breakdown of a fatty acid in the absence of oxygen. A fatty acid is any of the aliphatic monocarboxylic acids that can be liberated by hydrolysis from naturally occurring fats and oils. Fatty acids are predominantly straight-chain acids of 4 to 24 carbon atoms, which may be saturated or unsaturated; branched fatty acids and hydroxy fatty acids also occur, and very long chain acids of over 30 carbons are found in waxes.